simple sieve plate [GO:0097220] (cellular component) Note: Often located on an end wall of a sieve tube member. Unspecialized sieve areas may occur on other parts of the cell. Relationships: is a type of GO:0097218 Definition: A sieve plate that contains a single specialized sieve area. Sources: ISBN:0471738433, POC:curators